{
  "gene_symbol": "CEPT1",
  "term_label": "diacylglycerol cholinephosphotransferase activity",
  "term_id": "GO:0004142",
  "gene": "UniProtKB:Q9Y6K0",
  "gene_name": "Choline_ethanolaminephosphotransferase 1"
}